{
  "term_label": "glutamine-fructose-6-phosphate transaminase (isomerizing) activity",
  "gene_symbol": "GFPT1",
  "gene": "UniProtKB:Q06210",
  "gene_name": "Glutamine--fructose-6-phosphate aminotransferase [isomerizing] 1",
  "term_id": "GO:0004360"
}